{
  "term_id": "GO:0006487",
  "term_label": "protein N-linked glycosylation",
  "gene": "UniProtKB:Q9UQ53",
  "gene_name": "Alpha-1,3-mannosyl-glycoprotein 4-beta-N-acetylglucosaminyltransferase B",
  "gene_symbol": "MGAT4B"
}